{
  "gene": "UniProtKB:Q15398",
  "term_label": "regulation of mitotic cell cycle",
  "term_id": "GO:0007346",
  "gene_name": "Disks large-associated protein 5",
  "gene_symbol": "DLGAP5"
}